{
  "gene_name": "Zinc transporter 7",
  "gene": "UniProtKB:Q8NEW0",
  "term_id": "GO:0005385",
  "gene_symbol": "SLC30A7",
  "term_label": "zinc ion transmembrane transporter activity"
}